{
  "gene": "UniProtKB:Q9ULB5",
  "term_label": "calcium-dependent cell-cell adhesion",
  "gene_name": "Cadherin-7",
  "gene_symbol": "CDH7",
  "term_id": "GO:0016339"
}